{
  "gene": "UniProtKB:Q9H4A3",
  "gene_name": "Serine_threonine-protein kinase WNK1",
  "term_label": "regulation of monoatomic cation transmembrane transport",
  "gene_symbol": "WNK1",
  "term_id": "GO:1904062"
}